{
  "term_label": "regulation of cell population proliferation",
  "term_id": "GO:0042127",
  "gene_symbol": "STAT2",
  "gene": "UniProtKB:P52630",
  "gene_name": "Signal transducer and activator of transcription 2"
}